{
  "gene_name": "Numb-like protein",
  "gene_symbol": "NUMBL",
  "term_label": "Unknown molecular function",
  "term_id": "UNKNOWN:0001",
  "gene": "UniProtKB:Q9Y6R0"
}